{
  "term_id": "GO:0006882",
  "gene_symbol": "MT4",
  "term_label": "intracellular zinc ion homeostasis",
  "gene": "UniProtKB:P47944",
  "gene_name": "Metallothionein-4"
}